{
  "term_id": "GO:0000727",
  "gene_symbol": "CDC7",
  "term_label": "double-strand break repair via break-induced replication",
  "gene_name": "Cell division cycle 7-related protein kinase",
  "gene": "UniProtKB:O00311"
}